{
  "gene_name": "Thiosulfate sulfurtransferase_rhodanese-like domain-containing protein 3",
  "term_label": "Unknown biological process",
  "gene_symbol": "TSTD3",
  "gene": "UniProtKB:H0UI37",
  "term_id": "UNKNOWN:0002"
}